{
  "term_id": "GO:0005737",
  "term_label": "cytoplasm",
  "gene_symbol": "PAOX",
  "gene_name": "Peroxisomal N(1)-acetyl-spermine_spermidine oxidase",
  "gene": "UniProtKB:Q6QHF9"
}